glyoxal catabolic process [GO:1903190] (biological process) Also known as: glyoxal breakdown, glyoxal catabolism, glyoxal degradation Definition: The chemical reactions and pathways resulting in the breakdown of glyoxal. References: PMID:22523093, PMID:23651081 Sources: GOC:PARL, GOC:TermGenie, GOC:bf, GO_REF:0000068 Relationships: is a type of aldehyde catabolic process [GO:0046185]; is a type of glyoxal metabolic process [GO:1903189]